{
  "gene_symbol": "CASP2",
  "term_id": "GO:0005737",
  "gene": "UniProtKB:P42575",
  "term_label": "cytoplasm",
  "gene_name": "Caspase-2"
}